{
  "term_id": "GO:0016525",
  "gene_symbol": "ISM1",
  "term_label": "negative regulation of angiogenesis",
  "gene": "UniProtKB:B1AKI9",
  "gene_name": "Isthmin-1"
}